{
  "term_label": "nucleus",
  "gene_symbol": "CHM",
  "gene": "UniProtKB:P24386",
  "term_id": "GO:0005634",
  "gene_name": "Rab proteins geranylgeranyltransferase component A 1"
}